{
  "gene_symbol": "FOXK1",
  "term_id": "GO:0006357",
  "gene_name": "Forkhead box protein K1",
  "gene": "UniProtKB:P85037",
  "term_label": "regulation of transcription by RNA polymerase II"
}